{
  "term_id": "GO:0098978",
  "gene_name": "Protein bassoon",
  "term_label": "glutamatergic synapse",
  "gene_symbol": "BSN",
  "gene": "UniProtKB:Q9UPA5"
}